{
  "term_id": "UNKNOWN:0002",
  "gene_name": "Cytochrome P450 20A1",
  "gene_symbol": "CYP20A1",
  "gene": "UniProtKB:Q6UW02",
  "term_label": "Unknown biological process"
}